{
  "term_id": "GO:0007179",
  "term_label": "transforming growth factor beta receptor signaling pathway",
  "gene": "UniProtKB:O14793",
  "gene_name": "Growth_differentiation factor 8",
  "gene_symbol": "MSTN"
}